mesenchymal to epithelial transition involved in mesonephric renal vesicle formation [GO:0061271] (biological process) Sources: GOC:mtg_kidney_jan10 Definition: A transition where a mesenchymal cell establishes apical/basolateral polarity,forms intercellular adhesive junctions, synthesizes basement membrane components and becomes an epithelial cell that will contribute to the shaping of the mesonephric renal vesicle. Relationships: is a type of mesenchymal to epithelial transition involved in mesonephros morphogenesis [GO:0061261]; is a type of mesenchymal to epithelial transition involved in renal vesicle formation [GO:0072036]; is part of GO:0061262